{
  "gene_name": "Ras-related GTP-binding protein B",
  "gene": "UniProtKB:Q5VZM2",
  "term_id": "GO:1990131",
  "term_label": "Gtr1-Gtr2 GTPase complex",
  "gene_symbol": "RRAGB"
}